{
  "term_label": "signal transduction",
  "gene_symbol": "RIPK2",
  "gene": "UniProtKB:O43353",
  "term_id": "GO:0007165",
  "gene_name": "Receptor-interacting serine_threonine-protein kinase 2"
}